{
  "term_label": "antiviral innate immune response",
  "gene": "UniProtKB:Q9Y6K5",
  "gene_symbol": "OAS3",
  "gene_name": "2'-5'-oligoadenylate synthase 3",
  "term_id": "GO:0140374"
}